{
  "term_label": "syntaxin binding",
  "gene_name": "Vacuolar protein sorting-associated protein 52 homolog",
  "gene": "UniProtKB:Q8N1B4",
  "gene_symbol": "VPS52",
  "term_id": "GO:0019905"
}